{
  "gene_symbol": "USE1",
  "gene": "UniProtKB:Q9NZ43",
  "term_label": "SNAP receptor activity",
  "term_id": "GO:0005484",
  "gene_name": "Vesicle transport protein USE1"
}